type 4 neuropeptide Y receptor binding [GO:0031844] (molecular function) Relationships: is a type of neuropeptide Y receptor binding [GO:0031841] Also known as: pancreatic polypeptide receptor binding, type 4 neuropeptide Y receptor ligand Definition: Binding to a type 4 neuropeptide Y receptor. Sources: GOC:mah, GOC:nln